{
  "term_label": "Unknown cellular component",
  "term_id": "UNKNOWN:0003",
  "gene_name": "Uncharacterized protein C17orf67",
  "gene": "UniProtKB:Q0P5P2",
  "gene_symbol": "C17orf67"
}